{
  "gene": "UniProtKB:P24385",
  "term_label": "cyclin-dependent protein kinase holoenzyme complex",
  "gene_name": "G1_S-specific cyclin-D1",
  "gene_symbol": "CCND1",
  "term_id": "GO:0000307"
}